{
  "gene": "UniProtKB:Q969H8",
  "gene_name": "Myeloid-derived growth factor",
  "term_label": "positive regulation of endothelial cell proliferation",
  "gene_symbol": "MYDGF",
  "term_id": "GO:0001938"
}